{
  "term_id": "GO:0005634",
  "gene_name": "Zinc finger C3H1 domain-containing protein",
  "gene_symbol": "ZFC3H1",
  "term_label": "nucleus",
  "gene": "UniProtKB:O60293"
}